midchain alkane hydroxylase activity [GO:0080133] (MF) Relationships: is a type of GO:0016713 Definition: Catalysis of the conversion of an alkane to a secondary alcohol. References: PMID:17905869